CD8-positive, gamma-delta intraepithelial T cell differentiation [GO:0002305] (biological process) Sources: GOC:add, ISBN:0781735149 Definition: The process in which a precursor cell type acquires the specialized features of a CD8-positive, gamma-delta intraepithelial T cell. Intraepithelial T cells are found among epithelial cells in mucosal areas and have distinct phenotypes and developmental pathways. Also known as: CD8-positive, gamma-delta intraepithelial T lymphocyte differentiation, CD8-positive, gamma-delta intraepithelial T-cell differentiation, CD8-positive, gamma-delta intraepithelial T-lymphocyte differentiation, CD8-positive, gamma-delta intraepithelial T cell development Note: Note that immunologists typically use the word 'development' to refer to cells of B or T cell lineages undergoing the process that GO describes as 'cell differentiation'. Relationships: is a type of gamma-delta intraepithelial T cell differentiation [GO:0002304]